choline kinase activity [GO:0004103] (MF) Relationships: is a type of kinase activity [GO:0016301]; is a type of GO:0016773; is part of CDP-choline pathway [GO:0006657] Sources: EC:2.7.1.32, RHEA:12837 Definition: Catalysis of the reaction: ATP + choline = ADP + choline phosphate + 2 H+. Also known as: ATP:choline phosphotransferase activity, choline kinase (phosphorylating), choline phosphokinase activity, choline-ethanolamine kinase activity